B cell receptor complex [GO:0019815] (cellular component) Also known as: B lymphocyte receptor complex, B-cell receptor complex, B-lymphocyte receptor complex, BCR complex, immunoglobulin complex, membrane bound, B cell receptor accessory molecule complex, antibody Definition: An immunoglobulin complex that is present in the plasma membrane of B cells and that in its canonical form is composed of two identical immunoglobulin heavy chains and two identical immunoglobulin light chains and a signaling subunit, a heterodimer of the Ig-alpha and Ig-beta proteins. Note: Note that an immunoglobulin complex has the function of antigen binding if a suitable antigen is available. Subtypes: GO:0071737, IgD B cell receptor complex [GO:0071740], IgE B cell receptor complex [GO:0071744], GO:0071747, IgM B cell receptor complex [GO:0071755] Relationships: is a type of immunoglobulin complex [GO:0019814]; is a type of plasma membrane signaling receptor complex [GO:0098802] Sources: GOC:add, ISBN:0781735149